{
  "term_label": "unsaturated fatty acid biosynthetic process",
  "gene_symbol": "SCD5",
  "gene_name": "Stearoyl-CoA desaturase 5",
  "gene": "UniProtKB:Q86SK9",
  "term_id": "GO:0006636"
}